{
  "gene_name": "Zinc finger CCCH domain-containing protein 8",
  "term_label": "nucleoplasm",
  "term_id": "GO:0005654",
  "gene_symbol": "ZC3H8",
  "gene": "UniProtKB:Q8N5P1"
}